fasciculation of sensory neuron axon [GO:0097155] (biological process) References: PMID:18403711 Sources: GOC:lb Relationships: is a type of axonal fasciculation [GO:0007413] Definition: The collection of sensory neuron axons into a bundle of rods, known as a fascicle.